{
  "gene_name": "CAD protein",
  "gene": "UniProtKB:P27708",
  "term_label": "'de novo' pyrimidine nucleobase biosynthetic process",
  "term_id": "GO:0006207",
  "gene_symbol": "CAD"
}